{
  "gene": "UniProtKB:O15050",
  "term_id": "UNKNOWN:0002",
  "gene_symbol": "TRANK1",
  "term_label": "Unknown biological process",
  "gene_name": "TPR and ankyrin repeat-containing protein 1"
}